{
  "gene": "UniProtKB:P45877",
  "gene_symbol": "PPIC",
  "term_label": "cyclosporin A binding",
  "gene_name": "Peptidyl-prolyl cis-trans isomerase C",
  "term_id": "GO:0016018"
}